{
  "term_label": "heme A biosynthetic process",
  "gene_name": "Protoheme IX farnesyltransferase, mitochondrial",
  "term_id": "GO:0006784",
  "gene": "UniProtKB:Q12887",
  "gene_symbol": "COX10"
}